regulation of intermediate filament depolymerization [GO:0030842] (biological process) Subtypes: negative regulation of intermediate filament depolymerization [GO:0030843], positive regulation of intermediate filament depolymerization [GO:0030844] Definition: Any process that modulates the frequency, rate or extent of the disassembly of intermediate filaments by the removal of monomers from a filament. Sources: GOC:mah Relationships: is a type of regulation of intermediate filament polymerization or depolymerization [GO:0045108]; is_a regulation of protein depolymerization [GO:1901879]; regulates intermediate filament depolymerization [GO:0045106]